{
  "gene": "UniProtKB:Q9H0U6",
  "gene_name": "Large ribosomal subunit protein uL18m",
  "gene_symbol": "MRPL18",
  "term_id": "UNKNOWN:0002",
  "term_label": "Unknown biological process"
}